regulation of germinal center formation [GO:0002634] (biological process) Relationships: is a type of regulation of adaptive immune response based on somatic recombination of immune receptors built from immunoglobulin superfamily domains [GO:0002822]; is_a regulation of anatomical structure morphogenesis [GO:0022603]; regulates germinal center formation [GO:0002467] Sources: GOC:add Definition: Any process that modulates the frequency, rate, or extent of germinal center formation. Subtypes: negative regulation of germinal center formation [GO:0002635], positive regulation of germinal center formation [GO:0002636]